{
  "term_label": "defense response to virus",
  "gene": "UniProtKB:Q9NRW3",
  "gene_name": "DNA dC-dU-editing enzyme APOBEC-3C",
  "gene_symbol": "APOBEC3C",
  "term_id": "GO:0051607"
}